{
  "term_label": "cell adhesion",
  "gene": "UniProtKB:Q92982",
  "gene_name": "Ninjurin-1",
  "gene_symbol": "NINJ1",
  "term_id": "GO:0007155"
}